{
  "gene": "UniProtKB:P51878",
  "term_label": "Unknown molecular function",
  "gene_name": "Caspase-5",
  "gene_symbol": "CASP5",
  "term_id": "UNKNOWN:0001"
}